regulation of bone resorption [GO:0045124] (biological process) Sources: GOC:ai Relationships: is a type of regulation of bone remodeling [GO:0046850]; regulates bone resorption [GO:0045453] Definition: Any process that modulates the frequency, rate or extent of bone tissue loss (resorption). Subtypes: negative regulation of bone resorption [GO:0045779], positive regulation of bone resorption [GO:0045780]